long-chain fatty-acyl-CoA catabolic process [GO:0036116] (biological process) Definition: The chemical reactions and pathways resulting in the breakdown of long-chain fatty-acyl-CoAs, any derivative of coenzyme A in which the sulfhydryl group is in a thioester linkage with a long-chain fatty-acyl group. A long-chain fatty acid has an aliphatic tail containing 13 to 22 carbons. Note: While there is not universal consensus on the lengths of short-, medium-, long- and very-long-chain fatty acids, the GO uses the definitions in ChEBI (see CHEBI:26666, CHEBI:59554, CHEBI:15904 and CHEBI:27283). Relationships: is a type of GO:0035336; is a type of GO:0036115 Also known as: long-chain fatty-acyl-CoA breakdown, long-chain fatty-acyl-CoA catabolism, long-chain fatty-acyl-CoA degradation Sources: GOC:pm